{
  "gene": "UniProtKB:P05154",
  "term_id": "GO:0004867",
  "term_label": "serine-type endopeptidase inhibitor activity",
  "gene_name": "Plasma serine protease inhibitor",
  "gene_symbol": "SERPINA5"
}